HLA-C specific inhibitory MHC class I receptor activity [GO:0030110] (molecular function) References: PMID:11929129, PMID:9368779 Sources: GOC:add, GOC:mah Relationships: is a type of inhibitory MHC class I receptor activity [GO:0032396] Definition: Combining with a MHC class I molecule of the HLA-C subclass to mediate signaling that inhibits activation of a lymphocyte.